protein targeting to lysosome [GO:0006622] (biological process) Subtypes: protein targeting to lysosome involved in chaperone-mediated autophagy [GO:0061740] Relationships: is a type of protein targeting to vacuole [GO:0006623]; is a type of GO:0007041; is a type of GO:0061462 Also known as: protein-lysosome targeting Sources: GOC:curators Definition: The process of directing proteins towards the lysosome using signals contained within the protein.